glucosamine biosynthetic process [GO:0006042] (biological process) Definition: The chemical reactions and pathways resulting in the formation of glucosamine (2-amino-2-deoxyglucopyranose), an aminodeoxysugar that occurs in combined form in chitin. Also known as: chitosamine biosynthesis, chitosamine biosynthetic process, glucosamine anabolism, glucosamine biosynthesis, glucosamine formation, glucosamine synthesis Relationships: is a type of glucosamine metabolic process [GO:0006041]; is_a glucosamine-containing compound biosynthetic process [GO:1901073] Sources: GOC:jl, ISBN:0198506732